D-serine catabolic process [GO:0036088] (biological process) Relationships: is a type of D-amino acid catabolic process [GO:0019478]; is a type of D-serine metabolic process [GO:0070178] Also known as: D-serine breakdown, D-serine catabolism, D-serine degradation Definition: The chemical reactions and pathways resulting in the breakdown of D-serine, the D-enantiomer of serine, i.e. (2S)-2-amino-3-hydroxypropanoic acid. Sources: GOC:imk